{
  "term_label": "GTPase activity",
  "term_id": "GO:0003924",
  "gene_name": "GPN-loop GTPase 1",
  "gene": "UniProtKB:Q9HCN4",
  "gene_symbol": "GPN1"
}